{
  "term_id": "GO:0007131",
  "gene_name": "Cyclin N-terminal domain-containing protein 1",
  "gene": "UniProtKB:Q8N815",
  "term_label": "reciprocal meiotic recombination",
  "gene_symbol": "CNTD1"
}